{
  "term_id": "GO:0019915",
  "gene_name": "Apolipoprotein C-IV",
  "gene_symbol": "APOC4",
  "term_label": "lipid storage",
  "gene": "UniProtKB:P55056"
}